positive regulation of hepatocyte growth factor receptor signaling pathway [GO:1902204] (biological process) Relationships: is a type of positive regulation of signal transduction [GO:0009967]; is a type of regulation of hepatocyte growth factor receptor signaling pathway [GO:1902202]; positively regulates GO:0048012 References: PMID:18819921 Sources: GOC:TermGenie Definition: Any process that activates or increases the frequency, rate or extent of hepatocyte growth factor receptor signaling pathway. Also known as: activation of HGF receptor signaling pathway, activation of HGF receptor signalling pathway, positive regulation of HGF receptor signaling pathway, positive regulation of HGF receptor signalling pathway, up regulation of HGF receptor signaling pathway, up regulation of HGF receptor signalling pathway, up regulation of hepatocyte growth factor receptor signaling pathway, up-regulation of HGF receptor signaling pathway, up-regulation of HGF receptor signalling pathway, up-regulation of hepatocyte growth factor receptor signaling pathway, upregulation of HGF receptor signaling pathway, upregulation of HGF receptor signalling pathway, upregulation of hepatocyte growth factor receptor signaling pathway, activation of Met signaling pathway, activation of hepatocyte growth factor receptor signaling pathway, positive regulation of Met signaling pathway, up regulation of Met signaling pathway, up-regulation of Met signaling pathway, upregulation of Met signaling pathway